{
  "gene_name": "Phosphatidylinositol 3,4,5-trisphosphate 3-phosphatase and dual-specificity protein phosphatase PTEN",
  "gene": "UniProtKB:P60484",
  "term_id": "GO:0005886",
  "term_label": "plasma membrane",
  "gene_symbol": "PTEN"
}